{
  "gene_name": "PAK4-inhibitor INKA2",
  "gene": "UniProtKB:Q9NTI7",
  "gene_symbol": "INKA2",
  "term_label": "protein kinase binding",
  "term_id": "GO:0019901"
}